{
  "gene_symbol": "BCO1",
  "gene": "UniProtKB:Q9HAY6",
  "term_label": "carotene catabolic process",
  "term_id": "GO:0016121",
  "gene_name": "Beta,beta-carotene 15,15'-dioxygenase"
}